{
  "gene_symbol": "VMP1",
  "gene": "UniProtKB:Q96GC9",
  "gene_name": "Vacuole membrane protein 1",
  "term_label": "endomembrane system",
  "term_id": "GO:0012505"
}